{
  "term_id": "GO:0098632",
  "gene": "UniProtKB:P56747",
  "gene_symbol": "CLDN6",
  "gene_name": "Claudin-6",
  "term_label": "cell-cell adhesion mediator activity"
}